{
  "gene_name": "Ankyrin repeat and LEM domain-containing protein 1",
  "gene_symbol": "ANKLE1",
  "term_label": "DNA endonuclease activity",
  "term_id": "GO:0004520",
  "gene": "UniProtKB:Q8NAG6"
}